{
  "gene_symbol": "RPS4Y1",
  "term_id": "GO:0006412",
  "gene_name": "Small ribosomal subunit protein eS4, Y isoform 1",
  "gene": "UniProtKB:P22090",
  "term_label": "translation"
}